stereocilia ankle link complex [GO:0002142] (cellular component) References: PMID:16775142 Relationships: is_a protein-containing complex [GO:0032991]; is part of stereocilia ankle link [GO:0002141] Definition: A complex of proteins that connect growing stereocilia in developing cochlear hair cells, composed of Vlgr1, usherin, vezatin, and whirlin.